{
  "term_label": "integrin binding",
  "gene_name": "Integrin beta-2",
  "gene_symbol": "ITGB2",
  "gene": "UniProtKB:P05107",
  "term_id": "GO:0005178"
}